cell-cell contact zone [GO:0044291] (cellular component) Sources: NIF_Subcellular:sao1299635018 Subtypes: GO:0014704, peg and socket contact [GO:0044286] Also known as: cell cell contact zone Definition: Extended zone of intimate apposition between two cells containing one or more types of intercellular junctions, e.g., the intercalated disk of muscle. Relationships: is a type of GO:0005911